terminal web assembly [GO:1902896] (biological process) Relationships: is a type of cortical actin cytoskeleton organization [GO:0030866]; is a type of membraneless organelle assembly [GO:0140694] Definition: The aggregation, arrangement and bonding together of a set of components to form a terminal web. References: PMID:21949650 Sources: GOC:TermGenie, GOC:kmv, GO_REF:0000079 Also known as: terminal web formation